{
  "gene_name": "E3 ubiquitin-protein ligase RNF5",
  "gene_symbol": "RNF5",
  "term_id": "GO:0044390",
  "term_label": "ubiquitin-like protein conjugating enzyme binding",
  "gene": "UniProtKB:Q99942"
}